{
  "gene_name": "GATOR complex protein WDR24",
  "term_label": "cellular response to amino acid starvation",
  "gene": "UniProtKB:Q96S15",
  "term_id": "GO:0034198",
  "gene_symbol": "WDR24"
}